BIM-BCL-2 complex [GO:0097141] (cellular component) Relationships: is a type of Bcl-2 family protein complex [GO:0097136] Definition: A heterodimeric protein complex consisting of BIM and BCL-2, members of the Bcl-2 family of anti- and proapoptotic regulators. References: PMID:14634621 Sources: GOC:so